{
  "term_label": "proteolysis involved in protein catabolic process",
  "term_id": "GO:0051603",
  "gene_symbol": "RNF123",
  "gene": "UniProtKB:Q5XPI4",
  "gene_name": "E3 ubiquitin-protein ligase RNF123"
}